{
  "gene": "UniProtKB:Q06643",
  "gene_symbol": "LTB",
  "gene_name": "Lymphotoxin-beta",
  "term_label": "positive regulation of canonical NF-kappaB signal transduction",
  "term_id": "GO:0043123"
}